{
  "term_id": "GO:0005525",
  "term_label": "GTP binding",
  "gene_symbol": "RAB11B",
  "gene_name": "Ras-related protein Rab-11B",
  "gene": "UniProtKB:Q15907"
}